bacteriocin immunity [GO:0030153] (biological process) Definition: A process that mediates resistance to a bacteriocin: any of a heterogeneous group of polypeptide antibiotics that are secreted by certain bacterial strains and are able to kill cells of other susceptible (frequently related) strains after adsorption at specific receptors on the cell surface. They include the colicins, and their mechanisms of action vary. Sources: GOC:mah, ISBN:0198506732 Relationships: is a type of toxin metabolic process [GO:0009404]